{
  "gene_symbol": "DOCK3",
  "term_label": "cytoplasm",
  "term_id": "GO:0005737",
  "gene": "UniProtKB:Q8IZD9",
  "gene_name": "Dedicator of cytokinesis protein 3"
}